{
  "term_label": "Unknown cellular component",
  "gene_symbol": "CCDC168",
  "term_id": "UNKNOWN:0003",
  "gene_name": "Leucine-rich repeat transmembrane protein CCDC168",
  "gene": "UniProtKB:Q8NDH2"
}